isopentadecanoic acid binding [GO:1904769] (molecular function) References: PMID:19828452 Sources: GOC:TermGenie, GOC:kmv, GO_REF:0000067 Also known as: 13-methylmyristic acid binding Definition: Binding to isopentadecanoic acid. Relationships: is_a long-chain fatty acid binding [GO:0036041]